cerebellar molecular layer maturation [GO:0021690] (biological process) Sources: GOC:cls, GOC:dgh, GOC:dph, GOC:jid, GO_REF:0000021 Definition: A developmental process, independent of morphogenetic (shape) change, that is required for the cerebellar molecular layer to attain its fully functional state. The molecular layer is the outermost layer of the cerebellar cortex. It contains the parallel fibers of the granule cells, interneurons such as stellate and basket cells, and the dendrites of the underlying Purkinje cells. Relationships: is a type of anatomical structure maturation [GO:0071695]; BFO_0000050 cerebellar molecular layer development [GO:0021679]; is part of cerebellar cortex maturation [GO:0021699]